erythrocyte clearance [GO:0034102] (BP) Relationships: is a type of GO:0048771; is part of erythrocyte homeostasis [GO:0034101] Note: Note that this term is intended for annotation of self-gene products that lead to elimination of erythrocytes without the involvement of a symbiont. Definition: The selective elimination of erythrocytes from the body by autoregulatory mechanisms. Regulation: regulated by regulation of erythrocyte clearance [GO:0034106]; negatively regulated by GO:0034107; RO_0002213 by positive regulation of erythrocyte clearance [GO:0034108] Also known as: RBC clearance, red blood cell clearance, neocytolysis References: PMID:12905029, PMID:14754397 Sources: GOC:add